{
  "gene_symbol": "IGKV3-15",
  "gene": "UniProtKB:P01624",
  "term_id": "UNKNOWN:0001",
  "gene_name": "Immunoglobulin kappa variable 3-15",
  "term_label": "Unknown molecular function"
}